{
  "gene": "UniProtKB:A6NE02",
  "term_id": "UNKNOWN:0001",
  "gene_symbol": "BTBD17",
  "term_label": "Unknown molecular function",
  "gene_name": "BTB_POZ domain-containing protein 17"
}